{
  "gene_name": "Large ribosomal subunit protein eL38",
  "term_label": "structural constituent of ribosome",
  "term_id": "GO:0003735",
  "gene_symbol": "RPL38",
  "gene": "UniProtKB:P63173"
}